{
  "gene_symbol": "FAM47A",
  "term_id": "UNKNOWN:0003",
  "gene": "UniProtKB:Q5JRC9",
  "gene_name": "Protein FAM47A",
  "term_label": "Unknown cellular component"
}